regulation of protein localization to cell tip [GO:1903066] (biological process) Definition: Any process that modulates the frequency, rate or extent of protein localization to cell tip. Subtypes: GO:0062107, GO:1903067, positive regulation of protein localization to cell tip [GO:1903068], regulation of protein localization to cell cortex of cell tip [GO:1990895] References: PMID:24554432 Sources: GOC:TermGenie, GO_REF:0000058 Relationships: is a type of regulation of protein localization [GO:0032880]; regulates protein localization to cell tip [GO:1990151] Also known as: regulation of protein localisation to cell tip